deacetylase activity [GO:0019213] (molecular function) Subtypes: N-acetylglucosaminylphosphatidylinositol deacetylase activity [GO:0000225], chitin deacetylase activity [GO:0004099], N-acetylglucosamine-6-phosphate deacetylase activity [GO:0008448], acetylornithine deacetylase activity [GO:0008777], protein lysine deacetylase activity [GO:0033558], steryl deacetylase activity [GO:0034084], N-acetylglucosaminylinositol deacetylase activity [GO:0035595], acetoxybutynylbithiophene deacetylase activity [GO:0047373], methylumbelliferyl-acetate deacetylase activity [GO:0047374], GO:0047375, GO:0047377, N-acetylgalactosamine-6-phosphate deacetylase activity [GO:0047419], 4-acetamidobutyrate deacetylase activity [GO:0047573], 4-acetamidobutyryl-CoA deacetylase activity [GO:0047574], GO:0047593, GO:0047609, GO:0047610, acetylspermidine deacetylase activity [GO:0047611], GO:0047739, N-acetyl-beta-alanine deacetylase activity [GO:0050117], N-acetyldiaminopimelate deacetylase activity [GO:0050118], N-acetylglucosamine deacetylase activity [GO:0050119], O-acetyl-ADP-ribose deacetylase activity [GO:0061463], GO:0102140 Definition: Catalysis of the hydrolysis of an acetyl group from a substrate molecule. Sources: GOC:jl Relationships: is a type of deacylase activity [GO:0160215] Regulation: positively regulated by positive regulation of deacetylase activity [GO:0090045]; regulated by GO:0150065